{
  "gene_symbol": "LOC128966728",
  "gene_name": "Uncharacterized protein",
  "term_id": "GO:0005886",
  "term_label": "plasma membrane",
  "gene": "UniProtKB:A0A0G2JMM0"
}